positive regulation of base-excision repair [GO:1905053] (biological process) Relationships: is a type of positive regulation of DNA repair [GO:0045739]; is a type of regulation of base-excision repair [GO:1905051]; positively regulates base-excision repair [GO:0006284] Also known as: positive regulation of BER, up regulation of BER, up regulation of base-excision repair, up-regulation of BER, up-regulation of base-excision repair, upregulation of BER, upregulation of base-excision repair, activation of BER, activation of base-excision repair Definition: Any process that activates or increases the frequency, rate or extent of base-excision repair. References: PMID:18973764 Sources: GOC:TermGenie, GOC:ah, GO_REF:0000058